{
  "gene_name": "Probable E3 ubiquitin-protein ligase HERC6",
  "gene": "UniProtKB:Q8IVU3",
  "term_id": "GO:0016567",
  "term_label": "protein ubiquitination",
  "gene_symbol": "HERC6"
}